symbiont-mediated disruption of host tissue [GO:0141146] (biological process) Definition: The process in which an organism effects a change that impairs the structure or function of a host tissue. This can occur via the disruption of the extracellular matrix, or the detachment of cells from the extracellular matrix, or the dissociation of the cells composing that tissue. The host is defined as the larger of the organisms involved in a symbiotic interaction. References: PMID:11982763, PMID:14651638, PMID:26355030 Also known as: cytopathogenic effect Relationships: is a type of symbiont-mediated disruption of host anatomical structure [GO:0052111] Subtypes: symbiont-mediated disruption of host mucosa [GO:0141139]